{
  "term_id": "GO:0000981",
  "gene_symbol": "ZNF718",
  "term_label": "DNA-binding transcription factor activity, RNA polymerase II-specific",
  "gene_name": "Zinc finger protein 718",
  "gene": "UniProtKB:Q3SXZ3"
}